{
  "gene": "UniProtKB:Q8NFT2",
  "gene_name": "Metalloreductase STEAP2",
  "term_label": "plasma membrane",
  "gene_symbol": "STEAP2",
  "term_id": "GO:0005886"
}